{
  "term_id": "GO:0005739",
  "gene": "UniProtKB:Q86U28",
  "gene_name": "Iron-sulfur cluster assembly 2 homolog, mitochondrial",
  "gene_symbol": "ISCA2",
  "term_label": "mitochondrion"
}